{
  "gene": "UniProtKB:Q9UJT1",
  "term_id": "GO:0000278",
  "term_label": "mitotic cell cycle",
  "gene_symbol": "TUBD1",
  "gene_name": "Tubulin delta chain"
}